{
  "gene_symbol": "LRRK2",
  "term_id": "GO:1900242",
  "gene_name": "Leucine-rich repeat serine_threonine-protein kinase 2",
  "term_label": "regulation of synaptic vesicle endocytosis",
  "gene": "UniProtKB:Q5S007"
}